{
  "gene": "UniProtKB:P08686",
  "term_id": "UNKNOWN:0003",
  "gene_symbol": "CYP21A2",
  "gene_name": "Steroid 21-hydroxylase",
  "term_label": "Unknown cellular component"
}